{
  "gene_symbol": "RPS6KA5",
  "term_id": "GO:0005654",
  "gene_name": "Ribosomal protein S6 kinase alpha-5",
  "gene": "UniProtKB:O75582",
  "term_label": "nucleoplasm"
}